{
  "gene_symbol": "FAM90A1",
  "gene": "UniProtKB:Q86YD7",
  "term_label": "Unknown biological process",
  "term_id": "UNKNOWN:0002",
  "gene_name": "Protein FAM90A1"
}